negative regulation of R7 cell differentiation [GO:0045677] (biological process) Also known as: down regulation of R7 differentiation, down-regulation of R7 differentiation, downregulation of R7 differentiation, negative regulation of R7 differentiation, inhibition of R7 differentiation Subtypes: negative regulation of sevenless signaling pathway [GO:0045873] Relationships: is a type of regulation of R7 cell differentiation [GO:0045676]; is a type of negative regulation of compound eye photoreceptor cell differentiation [GO:0110118]; negatively regulates R7 cell differentiation [GO:0045466] Sources: GOC:dph, GOC:go_curators, GOC:tb Definition: Any process that stops, prevents, or reduces the frequency, rate or extent of R7cell differentiation.